fatty acid omega-oxidation [GO:0010430] (biological process) References: PMID:16404574 Sources: MetaCyc:PWY-2724 Definition: A fatty acid oxidation process in which the methyl group at the end of the fatty acid molecule (the omega carbon) is first oxidized to a hydroxyl group, then to an oxo group, and finally to a carboxyl group. The long chain dicarboxylates derived from omega-oxidation then enter the beta-oxidation pathway for further degradation. Relationships: is a type of fatty acid oxidation [GO:0019395]